{
  "gene_name": "Sorting nexin-31",
  "term_id": "GO:0005769",
  "gene_symbol": "SNX31",
  "term_label": "early endosome",
  "gene": "UniProtKB:Q8N9S9"
}